lumenal side of transport vesicle membrane [GO:0098538] (cellular component) Sources: GOC:ab Subtypes: lumenal side of trans-Golgi network transport vesicle membrane [GO:0098540] Also known as: internal side of transport vesicle membrane Definition: The side (leaflet) of the transport vesicle membrane that faces the lumen. Relationships: is a type of lumenal side of membrane [GO:0098576]; is part of transport vesicle membrane [GO:0030658]